{
  "gene": "UniProtKB:O00462",
  "gene_name": "Beta-mannosidase",
  "gene_symbol": "MANBA",
  "term_label": "glycoprotein catabolic process",
  "term_id": "GO:0006516"
}